{
  "term_label": "Unknown cellular component",
  "gene_symbol": "HSD11B1L",
  "term_id": "UNKNOWN:0003",
  "gene": "UniProtKB:Q7Z5J1",
  "gene_name": "Hydroxysteroid 11-beta-dehydrogenase 1-like protein"
}